{
  "gene": "UniProtKB:P05111",
  "gene_name": "Inhibin alpha chain",
  "gene_symbol": "INHA",
  "term_id": "GO:0007178",
  "term_label": "cell surface receptor protein serine/threonine kinase signaling pathway"
}